{
  "gene_name": "Nucleoplasmin-2",
  "term_label": "nucleolus",
  "gene": "UniProtKB:Q86SE8",
  "gene_symbol": "NPM2",
  "term_id": "GO:0005730"
}